{
  "term_label": "protein import into mitochondrial matrix",
  "term_id": "GO:0030150",
  "gene_name": "GrpE protein homolog 1, mitochondrial",
  "gene_symbol": "GRPEL1",
  "gene": "UniProtKB:Q9HAV7"
}